{
  "term_label": "intracellular cholesterol transport",
  "gene_symbol": "STARD4",
  "gene_name": "StAR-related lipid transfer protein 4",
  "gene": "UniProtKB:Q96DR4",
  "term_id": "GO:0032367"
}